{
  "term_label": "rRNA pseudouridine synthesis",
  "gene": "UniProtKB:Q9NX24",
  "gene_symbol": "NHP2",
  "term_id": "GO:0031118",
  "gene_name": "H_ACA ribonucleoprotein complex subunit 2"
}